{
  "gene_name": "Cyclic nucleotide-gated cation channel alpha-3",
  "term_id": "GO:0060041",
  "gene_symbol": "CNGA3",
  "gene": "UniProtKB:Q16281",
  "term_label": "retina development in camera-type eye"
}